{
  "term_label": "cytoplasm",
  "gene": "UniProtKB:Q9Y2D0",
  "gene_name": "Carbonic anhydrase 5B, mitochondrial",
  "gene_symbol": "CA5B",
  "term_id": "GO:0005737"
}